{
  "gene_name": "Ladinin-1",
  "gene_symbol": "LAD1",
  "gene": "UniProtKB:O00515",
  "term_id": "UNKNOWN:0002",
  "term_label": "Unknown biological process"
}